{
  "term_label": "Unknown biological process",
  "term_id": "UNKNOWN:0002",
  "gene": "UniProtKB:Q8N412",
  "gene_symbol": "STPG2",
  "gene_name": "Sperm-tail PG-rich repeat-containing protein 2"
}